biogenic amine catabolic process [GO:0042402] (biological process) Subtypes: GO:0001695, polyamine catabolic process [GO:0006598], phenylethylamine catabolic process [GO:0019607], GO:0030419, GO:0042424, GO:0042426, octopamine catabolic process [GO:0046334], ethanolamine catabolic process [GO:0046336] Definition: The chemical reactions and pathways occurring at the level of individual cells resulting in the breakdown of biogenic amines, any of a group of naturally occurring, biologically active amines, such as norepinephrine, histamine, and serotonin, many of which act as neurotransmitters. Also known as: biogenic amine breakdown, biogenic amine catabolism, biogenic amine degradation Relationships: is a type of GO:0009310 Sources: GOC:go_curators, GOC:jl, ISBN:0198506732